{
  "gene": "UniProtKB:A1E959",
  "term_label": "nucleus",
  "term_id": "GO:0005634",
  "gene_name": "Odontogenic ameloblast-associated protein",
  "gene_symbol": "ODAM"
}